inhibitory C-type lectin receptor signaling pathway [GO:0002772] (biological process) Also known as: inhibitory C-type lectin receptor signalling pathway, Ly49 inhibitory receptor signaling pathway Definition: The series of molecular signals initiated by an extracellular ligand binding to an inhibitory C-type lectin receptor capable of inhibiting an immune effector process contributing to an immune response. References: PMID:15771571 Sources: GOC:add, ISBN:0781735149 Relationships: is a type of immune response-inhibiting cell surface receptor signaling pathway [GO:0002767]